{
  "gene_name": "Tumor necrosis factor receptor superfamily member 16",
  "gene_symbol": "NGFR",
  "term_label": "plasma membrane",
  "gene": "UniProtKB:P08138",
  "term_id": "GO:0005886"
}